{
  "gene_symbol": "NEMF",
  "gene": "UniProtKB:O60524",
  "gene_name": "Ribosome quality control complex subunit NEMF",
  "term_label": "RQC complex",
  "term_id": "GO:1990112"
}